{
  "gene_symbol": "CACNA2D4",
  "term_label": "voltage-gated calcium channel complex",
  "term_id": "GO:0005891",
  "gene_name": "Voltage-dependent calcium channel subunit alpha-2_delta-4",
  "gene": "UniProtKB:Q7Z3S7"
}